{
  "gene": "UniProtKB:O95196",
  "term_id": "GO:0045211",
  "term_label": "postsynaptic membrane",
  "gene_symbol": "CSPG5",
  "gene_name": "Chondroitin sulfate proteoglycan 5"
}